embryonic camera-type eye development [GO:0031076] (biological process) Definition: The process occurring during the embryonic phase whose specific outcome is the progression of the eye over time, from its formation to the mature structure. Relationships: is a type of camera-type eye development [GO:0043010]; is a type of embryonic organ development [GO:0048568] Sources: GOC:mah, GOC:mtg_sensu Regulation: regulated by regulation of embryonic camera-type eye development [GO:1902863]; negatively regulated by negative regulation of embryonic camera-type eye development [GO:1902864]; positively regulated by positive regulation of embryonic camera-type eye development [GO:1902865] Also known as: embryonic eye development